{
  "term_id": "GO:0000226",
  "term_label": "microtubule cytoskeleton organization",
  "gene": "UniProtKB:P78559",
  "gene_name": "Microtubule-associated protein 1A",
  "gene_symbol": "MAP1A"
}